{
  "gene_symbol": "ARL3",
  "gene_name": "ADP-ribosylation factor-like protein 3",
  "gene": "UniProtKB:P36405",
  "term_id": "GO:0060271",
  "term_label": "cilium assembly"
}